estrogen response element binding [GO:0034056] (molecular function) Relationships: is a type of GO:0000978 References: PMID:15036253, PMID:17975005 Sources: GOC:ecd Definition: Binding to an estrogen response element (ERE), a conserved sequence found in the promoters of genes whose expression is regulated in response to estrogen. Also known as: ERE binding